zygotic genome activation [GO:0141064] (biological process) Relationships: is_a positive regulation of gene expression [GO:0010628]; is part of maternal-to-zygotic transition of gene expression [GO:0160021] Definition: A process that contributes to the onset of de novo transcription from the zygotic genome as part of the maternal-to-zygote transition in gene expression. The zygote overcomes the silencing that has been established. The cause of this silencing could be due to several factors: chromatin modifications leading to repression, or lack of adequate transcription machinery. References: PMID:19204068, PMID:20808952 Also known as: ZGA